negative regulation of killing of cells of another organism [GO:0051711] (biological process) Sources: GOC:ai Relationships: is a type of negative regulation of cell killing [GO:0031342]; is a type of regulation of killing of cells of another organism [GO:0051709]; negatively regulates killing of cells of another organism [GO:0031640] Definition: Any process that stops, prevents, or reduces the frequency, rate or extent of the killing by an organism of cells in another organism. Subtypes: GO:0070955 Also known as: down regulation of killing of cells of another organism, down-regulation of killing of cells of another organism, downregulation of killing of cells of another organism, negative regulation of killing of cells of other organism, inhibition of killing of cells of another organism